cytoplasm protein quality control by the ubiquitin-proteasome system [GO:0071629] (biological process) Definition: The chemical reactions and pathways resulting in the breakdown of misfolded proteins in the cytoplasm, which are targeted to cytoplasmic proteasomes for degradation. References: PMID:20080635 Sources: GOC:mah, GOC:rb Relationships: is a type of GO:0043161; is a type of cytoplasm protein quality control [GO:0140455]; is part of cellular response to misfolded protein [GO:0071218] Also known as: cytoplasm-associated proteasomal ubiquitin-dependent protein breakdown, cytoplasm-associated proteasomal ubiquitin-dependent protein catabolism, cytoplasm-associated proteasomal ubiquitin-dependent protein degradation, ubiquitin-dependent catabolism of misfolded proteins by cytoplasm-associated proteasome Note: See also the biological process terms 'unfolded protein response ; GO:0030968' and 'retrograde protein transport, ER to cytosol ; GO:0030970'.